{
  "gene_name": "Palmitoyltransferase ZDHHC20",
  "term_label": "endoplasmic reticulum",
  "gene_symbol": "ZDHHC20",
  "term_id": "GO:0005783",
  "gene": "UniProtKB:Q5W0Z9"
}